{
  "term_label": "translation release factor activity, codon nonspecific",
  "gene": "UniProtKB:Q14197",
  "term_id": "GO:0016150",
  "gene_symbol": "MRPL58",
  "gene_name": "Large ribosomal subunit protein mL62"
}